double-stranded DNA binding [GO:0003690] (molecular function) Definition: Binding to double-stranded DNA. Sources: GOC:elh, GOC:vw Subtypes: GO:0003691, left-handed Z-DNA binding [GO:0003692], GO:0010385, mismatched DNA binding [GO:0030983], GO:0044729, GO:0061776, GO:0097100, DNA-DNA tethering activity [GO:0106260], sequence-specific double-stranded DNA binding [GO:1990837] Relationships: is a type of GO:0003677 Also known as: dsDNA binding